oligoxyloglucan reducing-end-specific cellobiohydrolase activity [GO:0033945] (molecular function) Also known as: oligoxyloglucan reducing end-specific cellobiohydrolase activity, oligoxyloglucan reducing-end cellobiohydrolase activity Relationships: is a type of hydrolase activity, hydrolyzing O-glycosyl compounds [GO:0004553] Sources: EC:3.2.1.150 Definition: Catalysis of the hydrolysis of cellobiose from the reducing end of xyloglucans consisting of a beta-(1->4) linked glucan carrying alpha-D-xylosyl groups on O-6 of the glucose residues. To be a substrate, the first residue must be unsubstituted, the second residue may bear a xylosyl group, whether further glycosylated or not, and the third residue, which becomes the new terminus by the action of the enzyme, is preferably xylosylated, but this xylose residue must not be further substituted.